{
  "gene_symbol": "NR0B1",
  "gene": "UniProtKB:P51843",
  "gene_name": "Nuclear receptor subfamily 0 group B member 1",
  "term_id": "GO:0016922",
  "term_label": "nuclear receptor binding"
}